{
  "gene_name": "Transient receptor potential cation channel subfamily M member 1",
  "gene_symbol": "TRPM1",
  "gene": "UniProtKB:Q7Z4N2",
  "term_label": "monoatomic cation transmembrane transport",
  "term_id": "GO:0098655"
}